{
  "term_label": "ubiquitin-dependent protein catabolic process",
  "term_id": "GO:0006511",
  "gene": "UniProtKB:P49427",
  "gene_symbol": "CDC34",
  "gene_name": "Ubiquitin-conjugating enzyme E2 R1"
}